quercetin O-glucoside biosynthetic process [GO:0033303] (biological process) Definition: The chemical reactions and pathways leading to the formation of O-glucosylated derivatives of quercetin. Sources: GOC:mah, MetaCyc:PWY-5321 Also known as: quercetin O-glucoside anabolism, quercetin O-glucoside biosynthesis, quercetin O-glucoside formation, quercetin O-glucoside synthesit Relationships: is a type of glycoside biosynthetic process [GO:0016138]; is a type of flavone biosynthetic process [GO:0051553]